{
  "gene": "UniProtKB:P59091",
  "term_label": "Unknown biological process",
  "gene_name": "Putative uncharacterized protein encoded by LINC00315",
  "gene_symbol": "LINC00315",
  "term_id": "UNKNOWN:0002"
}